cspyrone B1 biosynthetic process [GO:1900802] (biological process) Also known as: cspyrone B1 anabolism, cspyrone B1 biosynthesis, cspyrone B1 formation, cspyrone B1 synthesis Definition: The chemical reactions and pathways resulting in the formation of cspyrone B1. Sources: GOC:TermGenie, GOC:di Relationships: is a type of ketone biosynthetic process [GO:0042181]; is a type of secondary metabolite biosynthetic process [GO:0044550]; is a type of carboxylic acid biosynthetic process [GO:0046394]; is a type of GO:1901336